regulation of tolerance induction to self antigen [GO:0002649] (biological process) Sources: GOC:add Relationships: is a type of regulation of tolerance induction [GO:0002643]; RO_0002211 tolerance induction to self antigen [GO:0002513] Subtypes: negative regulation of tolerance induction to self antigen [GO:0002650], positive regulation of tolerance induction to self antigen [GO:0002651] Definition: Any process that modulates the frequency, rate, or extent of tolerance induction to self antigen.